{
  "term_label": "phospholipid metabolic process",
  "gene": "UniProtKB:Q32ZL2",
  "gene_symbol": "PLPPR5",
  "gene_name": "Phospholipid phosphatase-related protein type 5",
  "term_id": "GO:0006644"
}